{
  "gene": "UniProtKB:Q9Y6X1",
  "term_id": "GO:0030968",
  "gene_symbol": "SERP1",
  "gene_name": "Stress-associated endoplasmic reticulum protein 1",
  "term_label": "endoplasmic reticulum unfolded protein response"
}